negative regulation of granuloma formation [GO:0002632] (biological process) Also known as: down regulation of granuloma formation, down-regulation of granuloma formation, downregulation of granuloma formation, inhibition of granuloma formation Sources: GOC:add Relationships: is a type of regulation of granuloma formation [GO:0002631]; is_a negative regulation of chronic inflammatory response [GO:0002677]; is a type of negative regulation of immune effector process [GO:0002698]; negatively regulates granuloma formation [GO:0002432] Definition: Any process that stops, prevents, or reduces the frequency, rate, or extent of granuloma formation.